dihydrophloroglucinol hydrolase activity [GO:0018766] (MF) Sources: UM-BBD_reactionID:r0008 Relationships: is a type of hydrolase activity, acting on acid carbon-carbon bonds, in ketonic substances [GO:0016823] Definition: Catalysis of the reaction: dihydrophloroglucinol + OH- = 3-hydroxy-5-oxohexanoate.